{
  "gene": "UniProtKB:Q96EA4",
  "gene_symbol": "SPDL1",
  "term_label": "outer kinetochore",
  "term_id": "GO:0000940",
  "gene_name": "Protein Spindly"
}